{
  "gene": "UniProtKB:Q5TZA2",
  "gene_symbol": "CROCC",
  "gene_name": "Rootletin",
  "term_id": "GO:0005814",
  "term_label": "centriole"
}